{
  "gene": "UniProtKB:Q53TS8",
  "term_label": "Unknown molecular function",
  "gene_name": "Cation channel sperm-associated targeting subunit tau",
  "gene_symbol": "C2CD6",
  "term_id": "UNKNOWN:0001"
}